{
  "term_label": "Unknown cellular component",
  "gene_symbol": "FKBP9P1",
  "term_id": "UNKNOWN:0003",
  "gene_name": "Putative FK506-binding protein 9-like protein",
  "gene": "UniProtKB:Q75LS8"
}